{
  "gene_symbol": "CASP2",
  "gene_name": "Caspase-2",
  "gene": "UniProtKB:P42575",
  "term_label": "positive regulation of neuron apoptotic process",
  "term_id": "GO:0043525"
}